{
  "term_label": "cytoplasm",
  "term_id": "GO:0005737",
  "gene_name": "Protein misato homolog 1",
  "gene": "UniProtKB:Q9BUK6",
  "gene_symbol": "MSTO1"
}